{
  "gene_name": "Mitogen-activated protein kinase kinase kinase 9",
  "term_id": "GO:0004706",
  "gene_symbol": "MAP3K9",
  "term_label": "JUN kinase kinase kinase activity",
  "gene": "UniProtKB:P80192"
}